cell junction [GO:0030054] (cellular component) References: PMID:26820516, PMID:28096264 Sources: GOC:aruk, GOC:bc, GOC:mah, ISBN:0198506732 Definition: A cellular component that forms a specialized region of connection between two or more cells, or between a cell and the extracellular matrix, or between two membrane-bound components of a cell, such as flagella. Relationships: is a type of cellular anatomical structure [GO:0110165] Subtypes: synapse [GO:0045202], anchoring junction [GO:0070161], flagella connector [GO:0120118]